{
  "term_label": "Unknown molecular function",
  "gene_name": "Testis-expressed protein 29",
  "gene": "UniProtKB:Q8N6K0",
  "term_id": "UNKNOWN:0001",
  "gene_symbol": "TEX29"
}